upper tip-link density [GO:1990435] (cellular component) Definition: An electron-dense plaque at the upper end of a stereocilia tip link that provides the anchor in the stereocilia membrane on the side of the stereocilium where the tip link ends. References: PMID:19447093 Also known as: UTLD Relationships: is a type of GO:1990427